phosphatidylcholine transfer activity [GO:0120019] (molecular function) Relationships: is a type of phosphatidylcholine transporter activity [GO:0008525]; is a type of phospholipid transfer activity [GO:0120014]; has part phosphatidylcholine binding [GO:0031210] Definition: Removes phosphatidylcholine from a membrane or a monolayer lipid particle, transports it through the aqueous phase while protected in a hydrophobic pocket, and brings it to an acceptor membrane or lipid particle. References: PMID:20823909, PMID:24220498, PMID:25797198 Sources: GOC:krc Also known as: phosphatidylcholine carrier activity, intermembrane phosphatidylcholine transfer activity